{
  "term_label": "adherens junction organization",
  "gene": "UniProtKB:P55289",
  "gene_name": "Cadherin-12",
  "term_id": "GO:0034332",
  "gene_symbol": "CDH12"
}